inositol-2,4,5,6-tetrakisphosphate 5-phosphatase activity [GO:1990650] (molecular function) References: PMID:15316017 Sources: GOC:al Relationships: is a type of GO:0052743 Definition: Catalysis of the reaction: 1D-myo-inositol 2,4,5,6-tetrakisphosphate + H2O = 1D-myo-inositol 2,4,6-trisphosphate + phosphate.